positive regulation of response to tumor cell [GO:0002836] (biological process) Also known as: positive regulation of response to tumour cell, up regulation of response to tumor cell, up-regulation of response to tumor cell, upregulation of response to tumor cell, activation of response to tumor cell, stimulation of response to tumor cell Relationships: is a type of positive regulation of response to biotic stimulus [GO:0002833]; is a type of regulation of response to tumor cell [GO:0002834]; positively regulates response to tumor cell [GO:0002347] Subtypes: positive regulation of immune response to tumor cell [GO:0002839] Definition: Any process that activates or increases the frequency, rate, or extent of a response to tumor cell. Sources: GOC:add